{
  "term_id": "GO:0043596",
  "gene_name": "Protein MCM10 homolog",
  "gene_symbol": "MCM10",
  "gene": "UniProtKB:Q7L590",
  "term_label": "nuclear replication fork"
}